type I interferon receptor activity [GO:0004905] (molecular function) Relationships: is a type of interferon receptor activity [GO:0004904]; BFO_0000050 type I interferon-mediated signaling pathway [GO:0060337]; has part GO:0019962 Definition: Combining with a type I interferon and transmitting the signal from one side of the membrane to the other to initiate a change in cell activity. Type I interferons include the interferon-alpha, beta, delta, epsilon, zeta, kappa, tau, and omega gene families. References: PMID:15546383, PMID:16681834 Sources: GOC:add, GOC:signaling, ISBN:0126896631 Also known as: type I IFN receptor activity, interferon-alpha receptor activity, interferon-alpha/beta receptor activity, interferon-beta receptor activity, interferon-delta receptor activity, interferon-epsilon receptor activity, interferon-kappa receptor activity, interferon-omega receptor activity, interferon-tau receptor activity, interferon-zeta receptor activity